{
  "term_id": "UNKNOWN:0001",
  "term_label": "Unknown molecular function",
  "gene_name": "Protein FAM43A",
  "gene": "UniProtKB:Q8N2R8",
  "gene_symbol": "FAM43A"
}